{
  "term_id": "GO:0005509",
  "gene_symbol": "CALML6",
  "term_label": "calcium ion binding",
  "gene_name": "Calmodulin-like protein 6",
  "gene": "UniProtKB:Q8TD86"
}